{
  "gene": "UniProtKB:Q8N4H5",
  "term_id": "UNKNOWN:0001",
  "gene_symbol": "TOMM5",
  "term_label": "Unknown molecular function",
  "gene_name": "Mitochondrial import receptor subunit TOM5 homolog"
}